primary endosperm nucleus [GO:0048353] (cellular component) Sources: ISBN:0471245208 Relationships: is a type of nucleus [GO:0005634] Definition: Nucleus resulting from the fusion of the male gamete and two polar nuclei in the central cell of the embryo sac.